positive regulation of receptor-mediated endocytosis [GO:0048260] (biological process) Sources: GOC:go_curators, GOC:tb Subtypes: positive regulation of receptor internalization [GO:0002092], positive regulation of receptor-mediated endocytosis involved in cholesterol transport [GO:1905602], positive regulation of clathrin-dependent endocytosis [GO:2000370] Definition: Any process that activates or increases the frequency, rate or extent of receptor mediated endocytosis, the uptake of external materials by cells, utilizing receptors to ensure specificity of transport. Relationships: is a type of positive regulation of endocytosis [GO:0045807]; is a type of regulation of receptor-mediated endocytosis [GO:0048259]; RO_0002213 receptor-mediated endocytosis [GO:0006898] Also known as: positive regulation of receptor mediated endocytosis, up regulation of receptor mediated endocytosis, up-regulation of receptor mediated endocytosis, upregulation of receptor mediated endocytosis, activation of receptor mediated endocytosis, stimulation of receptor mediated endocytosis